regulation of ethanol catabolic process [GO:1900065] (biological process) Definition: Any process that modulates the frequency, rate or extent of ethanol catabolic process. Also known as: regulation of ethanol breakdown, regulation of ethanol catabolism, regulation of ethanol degradation Relationships: is a type of regulation of alcohol catabolic process [GO:1900419]; regulates ethanol catabolic process [GO:0006068] References: PMID:10608811, PMID:7760841 Sources: GOC:TermGenie Subtypes: positive regulation of ethanol catabolic process [GO:1900066]